{
  "gene": "UniProtKB:Q9UIH9",
  "gene_name": "Krueppel-like factor 15",
  "gene_symbol": "KLF15",
  "term_label": "RNA polymerase II cis-regulatory region sequence-specific DNA binding",
  "term_id": "GO:0000978"
}